{
  "term_label": "ESCRT III complex",
  "gene_symbol": "CHMP4C",
  "gene_name": "Charged multivesicular body protein 4c",
  "term_id": "GO:0000815",
  "gene": "UniProtKB:Q96CF2"
}